{
  "term_label": "Unknown cellular component",
  "gene_symbol": "FRRS1L",
  "term_id": "UNKNOWN:0003",
  "gene": "UniProtKB:Q9P0K9",
  "gene_name": "DOMON domain-containing protein FRRS1L"
}